{
  "term_label": "Unknown cellular component",
  "term_id": "UNKNOWN:0003",
  "gene": "UniProtKB:A0A1B0GV22",
  "gene_symbol": "FAM236B",
  "gene_name": "Protein FAM236B"
}